{
  "term_id": "UNKNOWN:0002",
  "gene_symbol": "OR4A5",
  "gene": "UniProtKB:Q8NH83",
  "term_label": "Unknown biological process",
  "gene_name": "Olfactory receptor 4A5"
}